{
  "term_id": "GO:0005739",
  "term_label": "mitochondrion",
  "gene_symbol": "ECH1",
  "gene_name": "Delta(3,5)-Delta(2,4)-dienoyl-CoA isomerase, mitochondrial",
  "gene": "UniProtKB:Q13011"
}